{
  "gene": "UniProtKB:P38398",
  "term_label": "mitotic G2 DNA damage checkpoint signaling",
  "gene_name": "Breast cancer type 1 susceptibility protein",
  "term_id": "GO:0007095",
  "gene_symbol": "BRCA1"
}